myeloid dendritic cell antigen processing and presentation [GO:0002469] (biological process) Definition: The process in which a myeloid dendritic cell expresses antigen (peptide or lipid) on its cell surface in association with an MHC protein complex. Relationships: is_a dendritic cell antigen processing and presentation [GO:0002468] Regulation: regulated by regulation of myeloid dendritic cell antigen processing and presentation [GO:0002607]; negatively regulated by negative regulation of myeloid dendritic cell antigen processing and presentation [GO:0002608]; positively regulated by GO:0002609 References: PMID:15771591 Sources: GOC:add, ISBN:0781735149